{
  "gene_name": "5-hydroxytryptamine receptor 2B",
  "term_label": "phospholipase C-activating serotonin receptor signaling pathway",
  "term_id": "GO:0007208",
  "gene": "UniProtKB:P41595",
  "gene_symbol": "HTR2B"
}